{
  "gene_name": "Ragulator complex protein LAMTOR4",
  "term_label": "Ragulator complex",
  "term_id": "GO:0071986",
  "gene": "UniProtKB:Q0VGL1",
  "gene_symbol": "LAMTOR4"
}